{
  "gene": "UniProtKB:Q9ULZ9",
  "gene_symbol": "MMP17",
  "term_id": "GO:0004222",
  "term_label": "metalloendopeptidase activity",
  "gene_name": "Matrix metalloproteinase-17"
}